{
  "term_id": "GO:0019221",
  "gene": "UniProtKB:Q9HC73",
  "gene_symbol": "CRLF2",
  "term_label": "cytokine-mediated signaling pathway",
  "gene_name": "Cytokine receptor-like factor 2"
}